{
  "gene_symbol": "UBE2W",
  "term_id": "GO:0061631",
  "term_label": "ubiquitin conjugating enzyme activity",
  "gene_name": "Ubiquitin-conjugating enzyme E2 W",
  "gene": "UniProtKB:Q96B02"
}